nuclear periphery [GO:0034399] (cellular component) Sources: GOC:krc, GOC:mah Relationships: is a type of cellular anatomical structure [GO:0110165]; is part of nuclear lumen [GO:0031981] Definition: The portion of the nuclear lumen proximal to the inner nuclear membrane.